{
  "term_id": "GO:0005634",
  "gene_symbol": "NOS3",
  "term_label": "nucleus",
  "gene": "UniProtKB:P29474",
  "gene_name": "Nitric oxide synthase 3"
}